{
  "gene": "UniProtKB:Q8WWP7",
  "term_id": "UNKNOWN:0002",
  "gene_symbol": "GIMAP1",
  "term_label": "Unknown biological process",
  "gene_name": "GTPase IMAP family member 1"
}